photosystem II oxygen evolving complex assembly [GO:0010270] (biological process) Definition: The aggregation, arrangement and bonding together of a set of components to form the oxygen evolving complex (OEC) of photosystem II on a thylakoid membrane. The OEC protects the calcium-4 manganese-5 oxide cluster which is bound to the D1 and CP43 proteins. The exact protein composition of the OEC varies between cyanobacteria and plants, and in plants consists of three extrinsic nuclear-encoded polypeptides: PsbO, PsbP and PsbQ. References: PMID:16282331 Sources: GOC:aa Relationships: is a type of photosystem II assembly [GO:0010207] Also known as: OEC (PSII) ASSEMBLY